{
  "gene_name": "Protein FAM106A",
  "term_label": "Unknown cellular component",
  "term_id": "UNKNOWN:0003",
  "gene_symbol": "FAM106A",
  "gene": "UniProtKB:Q4KMX7"
}